somite rostral/caudal axis specification [GO:0032525] (biological process) Relationships: is a type of GO:0000578; is a type of anterior/posterior axis specification [GO:0009948]; is part of GO:0001756 References: PMID:16326386, PMID:17360776 Sources: GOC:bf Definition: The establishment, maintenance and elaboration of the rostro-caudal axis of a somite, prior to the morphological formation of a somite boundary. Also known as: somite rostrocaudal axis specification, somite rostrocaudal polarity